{
  "gene_name": "Zinc finger protein 623",
  "gene": "UniProtKB:O75123",
  "term_id": "GO:0000981",
  "term_label": "DNA-binding transcription factor activity, RNA polymerase II-specific",
  "gene_symbol": "ZNF623"
}